{
  "term_id": "GO:0008582",
  "term_label": "regulation of synaptic assembly at neuromuscular junction",
  "gene_symbol": "LIN7A",
  "gene": "UniProtKB:O14910",
  "gene_name": "Protein lin-7 homolog A"
}